negative regulation of plasma cell differentiation [GO:1900099] (biological process) Also known as: down regulation of plasma cell differentiation, down-regulation of plasma cell differentiation, downregulation of plasma cell differentiation, inhibition of plasma cell differentiation, down regulation of plasma cell development, down-regulation of plasma cell development, downregulation of plasma cell development, inhibition of plasma cell development, negative regulation of plasma cell development Relationships: is a type of negative regulation of immune effector process [GO:0002698]; is a type of negative regulation of B cell differentiation [GO:0045578]; is a type of GO:0050777; is a type of GO:1900098; negatively regulates plasma cell differentiation [GO:0002317] Sources: GOC:TermGenie Definition: Any process that stops, prevents or reduces the frequency, rate or extent of plasma cell differentiation.